{
  "gene": "UniProtKB:Q8NE09",
  "gene_symbol": "RGS22",
  "gene_name": "Regulator of G-protein signaling 22",
  "term_label": "cytoplasm",
  "term_id": "GO:0005737"
}